{
  "gene": "UniProtKB:P11684",
  "term_id": "GO:0005737",
  "gene_name": "Uteroglobin",
  "term_label": "cytoplasm",
  "gene_symbol": "SCGB1A1"
}